{
  "gene": "UniProtKB:Q86TY3",
  "term_label": "Unknown molecular function",
  "gene_symbol": "ARMH4",
  "term_id": "UNKNOWN:0001",
  "gene_name": "Armadillo-like helical domain-containing protein 4"
}